{
  "term_id": "GO:0098536",
  "term_label": "deuterosome",
  "gene_name": "Deuterosome assembly protein 1",
  "gene": "UniProtKB:Q05D60",
  "gene_symbol": "DEUP1"
}